protein C inhibitor-acrosin complex [GO:0033282] (CC) References: PMID:11120760, PMID:7521127 Sources: GOC:pr Relationships: is a type of serine protease inhibitor complex [GO:0097180]; is a type of membrane protein complex [GO:0098796]; is part of GO:0002080 Also known as: PCI-ACR complex, PCI-acrosin complex, SERPINA5-acrosin complex, plasma serine protease inhibitor-acrosin complex, serpin A5-acrosin complex Definition: A heterodimeric protein complex of protein C inhibitor (SERPINA5) and acrosin; formation of the complex inhibits the protease activity of acrosin.